{
  "term_label": "molecular adaptor activity",
  "gene_name": "Protein PAXX",
  "gene_symbol": "PAXX",
  "term_id": "GO:0060090",
  "gene": "UniProtKB:Q9BUH6"
}